{
  "term_id": "GO:0006631",
  "term_label": "fatty acid metabolic process",
  "gene": "UniProtKB:Q96CM8",
  "gene_name": "Medium-chain acyl-CoA ligase ACSF2, mitochondrial",
  "gene_symbol": "ACSF2"
}